{
  "gene_name": "Epiplakin",
  "gene": "UniProtKB:P58107",
  "term_label": "intermediate filament bundle assembly",
  "term_id": "GO:0045110",
  "gene_symbol": "EPPK1"
}